{
  "gene_symbol": "PRR20B",
  "term_label": "Unknown cellular component",
  "term_id": "UNKNOWN:0003",
  "gene": "UniProtKB:P86481",
  "gene_name": "Proline-rich protein 20B"
}